{
  "gene_symbol": "ZNF548",
  "gene_name": "Zinc finger protein 548",
  "term_id": "GO:0000978",
  "term_label": "RNA polymerase II cis-regulatory region sequence-specific DNA binding",
  "gene": "UniProtKB:Q8NEK5"
}